segmentation [GO:0035282] (biological process) Subtypes: somitogenesis [GO:0001756], blastoderm segmentation [GO:0007350], central nervous system segmentation [GO:0035283], brain segmentation [GO:0035284], appendage segmentation [GO:0035285], trunk segmentation [GO:0035290], GO:0061150 Relationships: is a type of regionalization [GO:0003002] Definition: The regionalization process that divides an organism or part of an organism into a series of semi-repetitive parts, or segments, often arranged along a longitudinal axis. References: PMID:10611687, PMID:9706689